{
  "gene_symbol": "TEX44",
  "gene_name": "Testis-expressed protein 44",
  "gene": "UniProtKB:Q53QW1",
  "term_label": "Unknown molecular function",
  "term_id": "UNKNOWN:0001"
}